{
  "gene_name": "Uncharacterized protein",
  "term_label": "Unknown cellular component",
  "gene_symbol": "A0A8V8TPW5",
  "gene": "UniProtKB:A0A8V8TPW5",
  "term_id": "UNKNOWN:0003"
}